abducens nerve formation [GO:0021599] (biological process) Definition: The process that gives rise to the abducens nerve. This process pertains to the initial formation of a structure from unspecified parts. The motor function of the abducens nerve is to contract the lateral rectus which results in abduction of the eye. Relationships: is a type of cranial nerve formation [GO:0021603]; is part of abducens nerve morphogenesis [GO:0021598] Sources: GOC:cls, GOC:dgh, GOC:dph, GOC:jid, GO_REF:0000021 Also known as: CN VI biosynthesis, CN VI formation